{
  "gene_name": "Myosin regulatory light chain 12B",
  "gene_symbol": "MYL12B",
  "gene": "UniProtKB:O14950",
  "term_id": "GO:0016460",
  "term_label": "myosin II complex"
}